{
  "term_id": "UNKNOWN:0003",
  "gene_symbol": "SLC22A6",
  "gene": "UniProtKB:Q4U2R8",
  "gene_name": "Solute carrier family 22 member 6",
  "term_label": "Unknown cellular component"
}